positive regulation of DNA-templated transcription initiation [GO:2000144] (BP) Definition: Any process that activates or increases the frequency, rate or extent of DNA-templated transcription initiation. Also known as: positive regulation of DNA-dependent transcription, initiation, positive regulation of DNA-templated transcription, initiation, positive regulation of initiation of DNA-dependent transcription, positive regulation of transcription initiation, DNA-dependent, transactivation, transcriptional transactivation Subtypes: positive regulation of transcription initiation by RNA polymerase II [GO:0060261] Sources: GOC:mah, GOC:txnOH Relationships: is a type of positive regulation of DNA-templated transcription [GO:0045893]; is a type of GO:2000142; positively regulates DNA-templated transcription initiation [GO:0006352]